{
  "term_label": "positive regulation of lamellipodium assembly",
  "gene": "UniProtKB:Q9H9L7",
  "gene_symbol": "AKIRIN1",
  "gene_name": "Akirin-1",
  "term_id": "GO:0010592"
}